ureidoglycolate lyase activity [GO:0050385] (molecular function) Also known as: (S)-ureidoglycolate urea-lyase (glyoxylate-forming), (S)-ureidoglycolate urea-lyase activity, ureidoglycolase activity, ureidoglycolatase activity, ureidoglycolate hydrolase activity Relationships: is_a amidine-lyase activity [GO:0016842] Definition: Catalysis of the reaction: (S)-ureidoglycolate = glyoxylate + urea. Note: Take care to annotate to the reaction, not simply by enzyme name. Note that the name "ureidoglycolate hydrolase" (listed as a synonym here) has variously been used to refer to two distinctly different enzymes. Both enzymes act on ureidoglycolate and produce glyoxylate, but the mechanism and reaction products are different. The "ureidoglycolate hydrolase" listed in the Enzyme commission (EC) is a ureidoglycolate amidohydrolase, releasing ammonia, (EC:3.5.3.19 ; GO:0004848). The "ureidoglycolate hydrolase" characterized in PMID:3915539 (published prior to the EC designation of EC:3.5.3.19) is a ureidoglycolate lyase, releasing urea (EC:4.3.2.3 ; GO:0050385). The inappropriate labelling of ureidoglycolate lyase as EC:3.5.3.19 has caused much confusion in the literature (see PMID:24107613). Take care to correctly annotate based on the reaction products, rather than name. Sources: EC:4.3.2.3, RHEA:11304